{
  "gene_name": "Protein C12orf4",
  "gene": "UniProtKB:Q9NQ89",
  "gene_symbol": "C12orf4",
  "term_id": "GO:0043304",
  "term_label": "regulation of mast cell degranulation"
}